{
  "term_label": "RNA polymerase II transcription regulatory region sequence-specific DNA binding",
  "gene_name": "LIM_homeobox protein Lhx3",
  "term_id": "GO:0000977",
  "gene_symbol": "LHX3",
  "gene": "UniProtKB:Q9UBR4"
}